{
  "term_label": "Unknown cellular component",
  "gene": "UniProtKB:Q8N1I8",
  "gene_name": "Putative uncharacterized protein encoded by CACTIN-AS1",
  "gene_symbol": "CACTIN-AS1",
  "term_id": "UNKNOWN:0003"
}